{
  "gene_symbol": "ARL6",
  "term_id": "GO:0061512",
  "term_label": "protein localization to cilium",
  "gene": "UniProtKB:Q9H0F7",
  "gene_name": "ADP-ribosylation factor-like protein 6"
}